ATF1-ATF4 transcription factor complex [GO:1990590] (cellular component) References: PMID:12871976 Sources: GOC:bhm Definition: Transcription factor complex consisting of ATF1 and ATF4 subunits that is capable of binding to cAMP response element (CRE) (consensus: 5'-GTGACGT[AC][AG]-3') of the GRP78 (HSPA5) promoter. Involved in the ER stress response pathway. Note: An example of this is ATF1in human (P18846) in PMID:12871976 (inferred from physical interaction). Relationships: is a type of GO:0090575